{
  "gene_name": "Nuclear receptor subfamily 1 group I member 2",
  "term_label": "negative regulation of transcription by RNA polymerase II",
  "term_id": "GO:0000122",
  "gene_symbol": "NR1I2",
  "gene": "UniProtKB:O75469"
}